{
  "term_label": "Golgi apparatus",
  "gene_name": "Ubiquitin carboxyl-terminal hydrolase 32",
  "term_id": "GO:0005794",
  "gene": "UniProtKB:Q8NFA0",
  "gene_symbol": "USP32"
}